{
  "gene": "UniProtKB:P86790",
  "term_label": "vacuolar transport",
  "gene_name": "Vacuolar fusion protein CCZ1 homolog B",
  "gene_symbol": "CCZ1B",
  "term_id": "GO:0007034"
}